{
  "term_id": "GO:0000981",
  "gene_symbol": "BHLHE22",
  "gene_name": "Class E basic helix-loop-helix protein 22",
  "term_label": "DNA-binding transcription factor activity, RNA polymerase II-specific",
  "gene": "UniProtKB:Q8NFJ8"
}